{
  "term_label": "early endosome",
  "gene": "UniProtKB:Q14694",
  "gene_name": "Ubiquitin carboxyl-terminal hydrolase 10",
  "gene_symbol": "USP10",
  "term_id": "GO:0005769"
}